{
  "gene": "UniProtKB:P14324",
  "gene_symbol": "FDPS",
  "term_id": "GO:0045337",
  "term_label": "farnesyl diphosphate biosynthetic process",
  "gene_name": "Farnesyl pyrophosphate synthase"
}